inulinase activity [GO:0051670] (molecular function) Also known as: 2,1-beta-D-fructan fructanohydrolase activity, endo-inulinase activity, exoinulinase activity, indoinulinase activity, inulase activity Sources: EC:3.2.1.7 Relationships: is a type of hydrolase activity, hydrolyzing O-glycosyl compounds [GO:0004553] Definition: Catalysis of the endohydrolysis of 2,1-beta-D-fructosidic linkages in inulin.